forebrain ventricular zone progenitor cell division [GO:0021869] (BP) References: PMID:16226447 Sources: GOC:cls, GOC:dgh, GOC:dph, GOC:jid, GO_REF:0000021 Subtypes: ventricular zone neuroblast division [GO:0021847] Definition: The mitotic division of a basal progenitor giving rise to two neurons. Relationships: is a type of cell division [GO:0051301]; is part of cell proliferation in forebrain [GO:0021846]